water transmembrane transporter activity [GO:0005372] (molecular function) Sources: GOC:ai Relationships: is a type of GO:0022857; is part of GO:0006833 Definition: Enables the transfer of water (H2O) from one side of a membrane to the other. Subtypes: water channel activity [GO:0015250]